3'-phosphoadenylylselenate reductase activity [GO:0098624] (molecular function) Also known as: PAPSe reductase activity References: PMID:14723223 Definition: Catalysis of the reaction: 3'-phosphoadenylylselenate + NADPH = adenosine 3',5'-bisphosphate + selenite + NADP+ + H+. Relationships: is a type of GO:0016651